{
  "term_label": "keratinization",
  "term_id": "GO:0031424",
  "gene": "UniProtKB:P78385",
  "gene_name": "Keratin, type II cuticular Hb3",
  "gene_symbol": "KRT83"
}